{
  "gene_symbol": "KSR2",
  "gene_name": "Kinase suppressor of Ras 2",
  "term_id": "GO:0004672",
  "gene": "UniProtKB:Q6VAB6",
  "term_label": "protein kinase activity"
}